{
  "term_label": "Unknown cellular component",
  "term_id": "UNKNOWN:0003",
  "gene_name": "cAMP-specific 3',5'-cyclic phosphodiesterase 4C",
  "gene": "UniProtKB:Q08493",
  "gene_symbol": "PDE4C"
}